{
  "term_label": "small GTPase-mediated signal transduction",
  "gene_name": "Proto-oncogene vav",
  "gene_symbol": "VAV1",
  "gene": "UniProtKB:P15498",
  "term_id": "GO:0007264"
}